{
  "gene": "UniProtKB:Q9HAV7",
  "gene_name": "GrpE protein homolog 1, mitochondrial",
  "term_label": "PAM complex, Tim23 associated import motor",
  "term_id": "GO:0001405",
  "gene_symbol": "GRPEL1"
}